{
  "term_label": "single-stranded DNA binding",
  "gene_name": "Replication protein A 14 kDa subunit",
  "gene_symbol": "RPA3",
  "term_id": "GO:0003697",
  "gene": "UniProtKB:P35244"
}